{
  "term_label": "cellular response to nerve growth factor stimulus",
  "gene_name": "High affinity nerve growth factor receptor",
  "gene_symbol": "NTRK1",
  "term_id": "GO:1990090",
  "gene": "UniProtKB:P04629"
}